{
  "term_id": "GO:0008033",
  "term_label": "tRNA processing",
  "gene": "UniProtKB:Q9NXH9",
  "gene_name": "tRNA (guanine(26)-N(2))-dimethyltransferase",
  "gene_symbol": "TRMT1"
}